{
  "term_id": "GO:0005886",
  "gene": "UniProtKB:O43586",
  "gene_name": "Proline-serine-threonine phosphatase-interacting protein 1",
  "gene_symbol": "PSTPIP1",
  "term_label": "plasma membrane"
}